{
  "term_id": "GO:0007166",
  "term_label": "cell surface receptor signaling pathway",
  "gene_name": "TNF receptor-associated factor 3",
  "gene_symbol": "TRAF3",
  "gene": "UniProtKB:Q13114"
}